{
  "gene_name": "Disintegrin and metalloproteinase domain-containing protein 33",
  "gene": "UniProtKB:Q9BZ11",
  "term_id": "UNKNOWN:0003",
  "gene_symbol": "ADAM33",
  "term_label": "Unknown cellular component"
}